{
  "term_id": "UNKNOWN:0002",
  "gene": "UniProtKB:Q5XKR9",
  "gene_name": "Protein FAM104B",
  "gene_symbol": "FAM104B",
  "term_label": "Unknown biological process"
}